{
  "gene": "UniProtKB:Q13835",
  "term_label": "cadherin binding",
  "term_id": "GO:0045296",
  "gene_symbol": "PKP1",
  "gene_name": "Plakophilin-1"
}